{
  "gene_name": "Transcription factor 12",
  "term_label": "regulation of transcription by RNA polymerase II",
  "term_id": "GO:0006357",
  "gene_symbol": "TCF12",
  "gene": "UniProtKB:Q99081"
}